{
  "gene_name": "Bifunctional polynucleotide phosphatase_kinase",
  "gene_symbol": "PNKP",
  "gene": "UniProtKB:Q96T60",
  "term_id": "GO:0046404",
  "term_label": "ATP-dependent polydeoxyribonucleotide 5'-hydroxyl-kinase activity"
}